regulation of early endosome to recycling endosome transport [GO:1902954] (biological process) References: PMID:22621900 Sources: GOC:TermGenie, GOC:sjp, GO_REF:0000058 Subtypes: positive regulation of early endosome to recycling endosome transport [GO:1902955] Relationships: is_a regulation of intracellular transport [GO:0032386]; is a type of GO:0060627; regulates early endosome to recycling endosome transport [GO:0061502] Definition: Any process that modulates the frequency, rate or extent of early endosome to recycling endosome transport.